{
  "gene_symbol": "CCDC142",
  "term_id": "UNKNOWN:0002",
  "gene_name": "Coiled-coil domain-containing protein 142",
  "term_label": "Unknown biological process",
  "gene": "UniProtKB:Q17RM4"
}